RNA polymerase II CTD heptapeptide repeat modifying activity [GO:0140994] (MF) Also known as: RNA polymerase II CTD repeat modifying activity, RNA polymerase II large subunit CTD heptapeptide repeat modifying activity Relationships: is a type of GO:0140096; is part of regulation of transcription by RNA polymerase II [GO:0006357] Definition: A catalytic activity that acts on the RNA polymerase II large subunit CTD heptapeptide repeat (consensus YSPTSPS). Reversible modifications cof the RNA polymerase II CTD repeats contribute to regulation of RNA polymerase activity. Subtypes: RNA polymerase II CTD heptapeptide repeat kinase activity [GO:0008353], GO:0008420, RNA polymerase II CTD heptapeptide repeat peptidyl-prolyl isomerase activity [GO:0140838] Sources: GOC:pg